{
  "gene": "UniProtKB:Q9Y265",
  "gene_name": "RuvB-like 1",
  "gene_symbol": "RUVBL1",
  "term_id": "GO:0006338",
  "term_label": "chromatin remodeling"
}